negative regulation of complement-dependent cytotoxicity [GO:1903660] (biological process) Relationships: is a type of negative regulation of cell killing [GO:0031342]; is a type of GO:1903659; negatively regulates complement-dependent cytotoxicity [GO:0097278] Also known as: down regulation of complement-dependent cytotoxicity, down-regulation of complement-dependent cytotoxicity, downregulation of complement-dependent cytotoxicity, inhibition of complement-dependent cytotoxicity References: PMID:24280217 Sources: GOC:TermGenie, GO_REF:0000058 Definition: Any process that stops, prevents or reduces the frequency, rate or extent of complement-dependent cytotoxicity.